{
  "gene_name": "AT-rich interactive domain-containing protein 3A",
  "gene": "UniProtKB:Q99856",
  "term_id": "GO:0003677",
  "gene_symbol": "ARID3A",
  "term_label": "DNA binding"
}